{
  "term_id": "UNKNOWN:0001",
  "gene_symbol": "SCARA3",
  "term_label": "Unknown molecular function",
  "gene": "UniProtKB:Q6AZY7",
  "gene_name": "Scavenger receptor class A member 3"
}